{
  "term_id": "GO:0002767",
  "gene": "UniProtKB:Q99706",
  "gene_symbol": "KIR2DL4",
  "term_label": "immune response-inhibiting cell surface receptor signaling pathway",
  "gene_name": "Killer cell immunoglobulin-like receptor 2DL4"
}